{
  "gene_symbol": "ORAI3",
  "gene": "UniProtKB:Q9BRQ5",
  "gene_name": "Protein orai-3",
  "term_label": "store-operated calcium entry",
  "term_id": "GO:0002115"
}